{
  "gene_symbol": "EXOSC6",
  "gene_name": "Exosome complex component MTR3",
  "gene": "UniProtKB:Q5RKV6",
  "term_label": "nucleolus",
  "term_id": "GO:0005730"
}